{
  "gene_symbol": "CYP4F2",
  "gene": "UniProtKB:P78329",
  "term_label": "phylloquinone catabolic process",
  "gene_name": "Cytochrome P450 4F2",
  "term_id": "GO:0042376"
}